{
  "gene": "UniProtKB:Q9NQV6",
  "term_label": "transcription cis-regulatory region binding",
  "term_id": "GO:0000976",
  "gene_name": "PR domain zinc finger protein 10",
  "gene_symbol": "PRDM10"
}